{
  "term_id": "GO:0034553",
  "gene_symbol": "SDHAF3",
  "term_label": "mitochondrial respiratory chain complex II assembly",
  "gene": "UniProtKB:Q9NRP4",
  "gene_name": "Succinate dehydrogenase assembly factor 3, mitochondrial"
}